{
  "gene": "UniProtKB:P06396",
  "gene_name": "Gelsolin",
  "term_label": "phosphatidylinositol-4,5-bisphosphate binding",
  "term_id": "GO:0005546",
  "gene_symbol": "GSN"
}